3-dehydroquinate dehydratase activity [GO:0003855] (molecular function) Relationships: is a type of GO:0016836 Definition: Catalysis of the reaction: 3-dehydroquinate = 3-dehydroshikimate + H2O. Also known as: 3-dehydroquinase activity, 3-dehydroquinate hydro-lyase (3-dehydroshikimate-forming), 3-dehydroquinate hydro-lyase activity, 3-dehydroquinate hydrolase activity, 5-dehydroquinase activity, 5-dehydroquinate dehydratase activity, 5-dehydroquinate hydro-lyase activity, DHQase, dehydroquinase activity, dehydroquinate dehydratase activity Sources: EC:4.2.1.10, RHEA:21096